{
  "gene": "UniProtKB:Q15633",
  "gene_symbol": "TARBP2",
  "term_label": "RISC complex",
  "term_id": "GO:0016442",
  "gene_name": "RISC-loading complex subunit TARBP2"
}